{
  "term_label": "cytoplasm",
  "gene_symbol": "LRRC41",
  "gene_name": "Leucine-rich repeat-containing protein 41",
  "gene": "UniProtKB:Q15345",
  "term_id": "GO:0005737"
}